{
  "gene_name": "PDZ and LIM domain protein 7",
  "term_id": "GO:0061061",
  "term_label": "muscle structure development",
  "gene": "UniProtKB:Q9NR12",
  "gene_symbol": "PDLIM7"
}